{
  "gene_symbol": "SHOC1",
  "term_id": "GO:0003697",
  "gene": "UniProtKB:Q5VXU9",
  "gene_name": "Protein shortage in chiasmata 1 ortholog",
  "term_label": "single-stranded DNA binding"
}